{
  "gene": "UniProtKB:Q92696",
  "term_label": "Rab geranylgeranyltransferase activity",
  "gene_symbol": "RABGGTA",
  "term_id": "GO:0004663",
  "gene_name": "Geranylgeranyl transferase type-2 subunit alpha"
}